{
  "term_id": "GO:0000122",
  "gene_symbol": "MAGEA9",
  "gene": "UniProtKB:P43362",
  "term_label": "negative regulation of transcription by RNA polymerase II",
  "gene_name": "Melanoma-associated antigen 9"
}